{
  "term_id": "GO:0008239",
  "gene_symbol": "PRSS16",
  "gene_name": "Thymus-specific serine protease",
  "gene": "UniProtKB:Q9NQE7",
  "term_label": "dipeptidyl-peptidase activity"
}